adenine transport [GO:0015853] (biological process) Relationships: is_a GO:0006863 Subtypes: GO:0098702 Sources: GOC:go_curators, ISBN:0198506732 Definition: The directed movement of adenine, 6-aminopurine, into, out of or within a cell, or between cells, by means of some agent such as a transporter or pore. Also known as: adenine transmembrane transport